{
  "gene_symbol": "NSMCE4A",
  "gene_name": "Non-structural maintenance of chromosomes element 4 homolog A",
  "term_id": "GO:0006281",
  "gene": "UniProtKB:Q9NXX6",
  "term_label": "DNA repair"
}